{
  "term_id": "GO:0030552",
  "gene_symbol": "PRKAR2A",
  "term_label": "cAMP binding",
  "gene_name": "cAMP-dependent protein kinase type II-alpha regulatory subunit",
  "gene": "UniProtKB:P13861"
}